branching involved in labyrinthine layer morphogenesis [GO:0060670] (biological process) References: PMID:16916377 Sources: GOC:dph Relationships: is_a embryonic morphogenesis [GO:0048598]; is a type of GO:0061138; is part of GO:0060713 Definition: The process in which the branches of the fetal placental villi are generated and organized. The villous part of the placenta is called the labyrinth layer.